{
  "gene": "UniProtKB:P63244",
  "term_label": "protein kinase C binding",
  "gene_name": "Small ribosomal subunit protein RACK1",
  "gene_symbol": "RACK1",
  "term_id": "GO:0005080"
}